glucose-6-phosphate 1-epimerase activity [GO:0047938] (molecular function) Sources: EC:5.1.3.15, MetaCyc:GLUCOSE-6-PHOSPHATE-1-EPIMERASE-RXN Also known as: glucose-6 phosphate 1-epimerase activity, D-glucose-6-phosphate 1-epimerase activity Relationships: is_a GO:0016857 Definition: Catalysis of the reaction: alpha-D-glucose 6-phosphate = beta-D-glucose 6-phosphate.